cysteine-dependent adenosine diphosphate thiazole synthase activity [GO:0160205] (molecular function) Relationships: is a type of pentosyltransferase activity [GO:0016763] Definition: Catalysis of the reaction: [ADP-thiazole synthase]-L-cysteine + glycine + NAD(+) = [ADP-thiazole synthase]-dehydroalanine + ADP-5-ethyl-4-methylthiazole-2-carboxylate + 2 H(+) + 3 H2O + nicotinamide. Also known as: suicide thiamine thiazole synthase activity, ADP-thiazole synthase activity Sources: RHEA:55708